{
  "term_id": "GO:0110032",
  "term_label": "positive regulation of G2/MI transition of meiotic cell cycle",
  "gene_symbol": "CDC25C",
  "gene": "UniProtKB:P30307",
  "gene_name": "M-phase inducer phosphatase 3"
}